{
  "gene_name": "Zinc finger protein 354A",
  "gene": "UniProtKB:O60765",
  "term_id": "GO:0000981",
  "gene_symbol": "ZNF354A",
  "term_label": "DNA-binding transcription factor activity, RNA polymerase II-specific"
}